arugosin catabolic process [GO:1900586] (biological process) Definition: The chemical reactions and pathways resulting in the breakdown of arugosin. Also known as: arugosin breakdown, arugosin catabolism, arugosin degradation Sources: GOC:TermGenie, GOC:di Relationships: is a type of secondary metabolite catabolic process [GO:0090487]